hepatoblast differentiation [GO:0061017] (biological process) Relationships: is_a epithelial cell differentiation [GO:0030855]; is a type of GO:0048863; is part of liver development [GO:0001889] Definition: The process in which a relatively unspecialized cell acquires specialized features of a hepatoblast. A hepatoblast is a cell that retains the ability to divide and proliferate throughout life to provide progenitor cells that can differentiate into hepatocytes and cholangiocytes. References: PMID:15226394 Sources: GOC:dph